{
  "gene_name": "Glycine receptor subunit beta",
  "gene_symbol": "GLRB",
  "term_id": "GO:1902476",
  "gene": "UniProtKB:P48167",
  "term_label": "chloride transmembrane transport"
}